{
  "term_label": "chemokine activity",
  "gene_symbol": "CXCL10",
  "gene_name": "C-X-C motif chemokine 10",
  "gene": "UniProtKB:P02778",
  "term_id": "GO:0008009"
}